{
  "term_id": "GO:0051604",
  "gene_name": "Kallikrein-5",
  "gene": "UniProtKB:Q9Y337",
  "gene_symbol": "KLK5",
  "term_label": "protein maturation"
}